{
  "term_id": "GO:0099502",
  "term_label": "calcium-dependent activation of synaptic vesicle fusion",
  "gene_symbol": "SYT8",
  "gene_name": "Synaptotagmin-8",
  "gene": "UniProtKB:Q8NBV8"
}